regulation of establishment of endothelial barrier [GO:1903140] (biological process) References: PMID:24851274 Sources: GOC:TermGenie, GOC:als, GO_REF:0000058 Subtypes: negative regulation of establishment of endothelial barrier [GO:1903141], positive regulation of establishment of endothelial barrier [GO:1903142] Definition: Any process that modulates the frequency, rate or extent of establishment of endothelial barrier. Relationships: is a type of regulation of endothelial cell development [GO:1901550]; regulates establishment of endothelial barrier [GO:0061028]